{
  "term_label": "Unknown biological process",
  "gene": "UniProtKB:Q5VVY1",
  "term_id": "UNKNOWN:0002",
  "gene_name": "N-terminal Xaa-Pro-Lys N-methyltransferase 2",
  "gene_symbol": "NTMT2"
}